{
  "gene": "UniProtKB:Q96LX8",
  "term_id": "GO:0001228",
  "term_label": "DNA-binding transcription activator activity, RNA polymerase II-specific",
  "gene_symbol": "ZNF597",
  "gene_name": "Zinc finger protein 597"
}